{
  "gene_name": "Spermatogenesis associated 6-like protein",
  "term_label": "Unknown cellular component",
  "gene_symbol": "SPATA6L",
  "term_id": "UNKNOWN:0003",
  "gene": "UniProtKB:Q8N4H0"
}